mesonephric nephron tubule formation [GO:0061277] (biological process) Sources: GOC:mtg_kidney_jan10 Relationships: is a type of mesonephric tubule formation [GO:0072172]; is part of mesonephric nephron tubule morphogenesis [GO:0061240] Definition: The developmental process pertaining to the initial formation of a mesonephric nephron tubule from unspecified parts. A mesonephric nephron tubule is an epithelial tube that is part of a nephron in the mesonephros.